positive regulation of anterograde axonal transport of mitochondrion [GO:0061881] (biological process) Relationships: is a type of GO:0032388; is a type of GO:0061880; positively regulates anterograde axonal transport of mitochondrion [GO:0098957] Also known as: positive regulation of anterograde axon transport of mitochondria References: PMID:24302729 Definition: Any process that activates or increasesthe frequency, rate or extent of the directed movement of mitochondria along microtubules in axons away from the cell body and towards the presynapse.